RNA lariat debranching enzyme activity [GO:0008419] (molecular function) References: PMID:7519612 Regulation: RO_0002213 by RNA lariat debranching enzyme activator activity [GO:0061632] Relationships: is a type of GO:0016891 Definition: Catalysis of the hydrolysis of branched RNA structures that contain vicinal 2'-5'- and 3'-5'-phosphodiester bonds at a branch point nucleotide.